chemokine (C-C motif) ligand 19 signaling pathway [GO:0038115] (biological process) Note: The C-C chemokine CCL19 s a known agonist of the chemokine receptor type 7 (CCR7). Consider instead annotating to the child term 'CCL19-activated CCR7 signaling pathway ; GO:0038119'. Also known as: CCL19-mediated signaling pathway, chemokine (C-C motif) ligand 19 signalling pathway, C-C chemokine receptor type 7 signaling pathway Relationships: is a type of GO:0070098 Definition: The series of molecular signals initiated by the binding of the C-C chemokine CCL19 to its receptor on the surface of a target cell, and ending with the regulation of a downstream cellular process, e.g. transcription. References: PMID:15059845 Sources: GOC:nhn, GOC:signaling Subtypes: CCL19-activated CCR7 signaling pathway [GO:0038119]